{
  "term_label": "Unknown molecular function",
  "term_id": "UNKNOWN:0001",
  "gene_symbol": "SELENOV",
  "gene": "UniProtKB:P59797",
  "gene_name": "Selenoprotein V"
}